adiponectin-activated signaling pathway [GO:0033211] (biological process) Definition: The series of molecular signals initiated by adiponectin binding to its receptor on the surface of a cell, and ending with the regulation of a downstream cellular process, e.g. transcription. Relationships: is a type of hormone-mediated signaling pathway [GO:0009755]; is a type of cytokine-mediated signaling pathway [GO:0019221] Also known as: adiponectin-mediated signalling pathway, adipocytokine signaling pathway, adiponectin-mediated signaling pathway References: PMID:20536390 Sources: GOC:mah, GOC:signaling